{
  "term_label": "endoplasmic reticulum membrane",
  "gene": "UniProtKB:Q9H1X3",
  "gene_symbol": "DNAJC25",
  "gene_name": "DnaJ homolog subfamily C member 25",
  "term_id": "GO:0005789"
}